regulation of circadian sleep/wake cycle, wakefulness [GO:0010840] (biological process) Relationships: is a type of GO:0042749; RO_0002211 circadian sleep/wake cycle, wakefulness [GO:0042746] Definition: Any process that modulates the rate, frequency, or extent of the wakeful phase of the circadian sleep/wake cycle. The wakeful phase is the part of the circadian sleep/wake cycle where the organism is not asleep. Sources: GOC:dph, GOC:tb Subtypes: positive regulation of circadian sleep/wake cycle, wakefulness [GO:0010841], negative regulation of circadian sleep/wake cycle, wakefulness [GO:1904326]